{
  "gene_symbol": "EHD3",
  "term_id": "GO:0032456",
  "gene_name": "EH domain-containing protein 3",
  "term_label": "endocytic recycling",
  "gene": "UniProtKB:Q9NZN3"
}